7-hydroxymethyl chlorophyll a reductase activity [GO:0090415] (MF) References: PMID:21934147 Sources: GOC:kad, RHEA:53544 Relationships: is_a GO:0052592 Definition: Catalysis of the reaction: 7-hydroxymethyl chlorophyll a + 2 reduced ferredoxin + 2 H+ chlorophyll a + 2 oxidized ferredoxin + H2O.